{
  "term_label": "Unknown biological process",
  "gene_name": "Putative uncharacterized protein SPART-AS1",
  "gene": "UniProtKB:P0CW21",
  "gene_symbol": "SPART-AS1",
  "term_id": "UNKNOWN:0002"
}